{
  "term_id": "UNKNOWN:0003",
  "term_label": "Unknown cellular component",
  "gene_name": "Putative uncharacterized protein MED14OS",
  "gene_symbol": "MED14OS",
  "gene": "UniProtKB:P0DP75"
}